{
  "term_label": "Unknown molecular function",
  "gene_symbol": "ZNF106",
  "gene_name": "Zinc finger protein 106",
  "term_id": "UNKNOWN:0001",
  "gene": "UniProtKB:Q9H2Y7"
}